{
  "gene_symbol": "LOC107984156",
  "gene": "UniProtKB:A0A0G2JMH3",
  "term_id": "GO:0016192",
  "term_label": "vesicle-mediated transport",
  "gene_name": "ADP-ribosylation factor-like protein 17 C-terminal domain-containing protein"
}